{
  "term_label": "RNA polymerase II cis-regulatory region sequence-specific DNA binding",
  "gene": "UniProtKB:P53567",
  "gene_symbol": "CEBPG",
  "gene_name": "CCAAT_enhancer-binding protein gamma",
  "term_id": "GO:0000978"
}